{
  "gene": "UniProtKB:Q96I45",
  "gene_name": "Transmembrane protein 141",
  "term_label": "Unknown molecular function",
  "term_id": "UNKNOWN:0001",
  "gene_symbol": "TMEM141"
}